larval foraging behavior [GO:0035177] (biological process) Definition: The movement of a larva through a feeding substrate whilst feeding on food. Relationships: is_a larval behavior [GO:0030537]; is a type of foraging behavior [GO:0060756] Also known as: larval foraging behaviour References: PMID:12848927